{
  "term_id": "UNKNOWN:0002",
  "term_label": "Unknown biological process",
  "gene_name": "Leukemia NUP98 fusion partner 1",
  "gene": "UniProtKB:A1A4G5",
  "gene_symbol": "LNP1"
}